positive regulation of BMP signaling pathway [GO:0030513] (biological process) Definition: Any process that activates or increases the frequency, rate or extent of BMP signaling pathway activity. Sources: GOC:go_curators Also known as: positive regulation of BMP signalling pathway, positive regulation of bone morphogenetic protein signaling pathway, positive regulation of bone morphogenetic protein signalling pathway, up regulation of BMP signaling pathway, up-regulation of BMP signaling pathway, upregulation of BMP signaling pathway, activation of BMP signaling pathway, positive regulation of decapentaplegic receptor signaling pathway, positive regulation of decapentaplegic receptor signalling pathway, positive regulation of decapentaplegic signaling pathway, stimulation of BMP signaling pathway, positive regulation of BMP receptor signaling pathway Relationships: is a type of regulation of BMP signaling pathway [GO:0030510]; is a type of positive regulation of transmembrane receptor protein serine/threonine kinase signaling pathway [GO:0090100]; positively regulates GO:0030509